{
  "term_id": "GO:0016567",
  "term_label": "protein ubiquitination",
  "gene_symbol": "RNF208",
  "gene": "UniProtKB:Q9H0X6",
  "gene_name": "RING finger protein 208"
}